{
  "gene_symbol": "GIMAP1",
  "term_id": "GO:0003924",
  "term_label": "GTPase activity",
  "gene_name": "GTPase IMAP family member 1",
  "gene": "UniProtKB:Q8WWP7"
}